intramolecular phosphotransferase complex [GO:1990233] (cellular component) Relationships: is a type of catalytic complex [GO:1902494]; is part of GO:0005829 References: PMID:16540464 Sources: GOC:bhm Subtypes: phosphomannomutase complex [GO:1990232] Definition: A protein complex capable of catalyzing the transfer of a phosphate group from one position to another within a single molecule.